{
  "term_id": "UNKNOWN:0001",
  "gene": "UniProtKB:Q96M42",
  "gene_name": "Putative uncharacterized protein encoded by LINC00479",
  "term_label": "Unknown molecular function",
  "gene_symbol": "LINC00479"
}